{
  "term_label": "calcium ion binding",
  "gene_name": "Cytosolic phospholipase A2",
  "gene": "UniProtKB:P47712",
  "term_id": "GO:0005509",
  "gene_symbol": "PLA2G4A"
}